UDP-galactose biosynthetic process [GO:0052574] (BP) Definition: The chemical reactions and pathways resulting in the formation of UDP-D-galactose, a substance composed of D-galactose in glycosidic linkage with guanosine diphosphate. Relationships: is a type of GO:0009226; is a type of UDP-D-galactose metabolic process [GO:0052573] Sources: GOC:ai Also known as: UDP-D-galactopyranose biosynthesis, UDP-D-galactopyranose biosynthetic process, UDP-D-galactose biosynthesis, UDP-D-galactose biosynthetic process, UDP-alpha-D-galactose biosynthesis, UDP-galactose biosynthesis, uridine diphosphate galactose biosynthesis, uridine diphosphate galactose biosynthetic process